{
  "term_label": "transmembrane transporter binding",
  "gene_name": "Caveolin-1",
  "term_id": "GO:0044325",
  "gene": "UniProtKB:Q03135",
  "gene_symbol": "CAV1"
}